DNA binding domain binding [GO:0050692] (molecular function) Relationships: is a type of protein domain specific binding [GO:0019904] References: PMID:9682036 Also known as: DBD binding Definition: Binding to a protein's DNA binding domain (DBD).